{
  "term_id": "GO:0031625",
  "gene": "UniProtKB:O94955",
  "gene_symbol": "RHOBTB3",
  "term_label": "ubiquitin protein ligase binding",
  "gene_name": "Rho-related BTB domain-containing protein 3"
}